{
  "term_id": "UNKNOWN:0002",
  "gene": "UniProtKB:Q96CP2",
  "gene_symbol": "FLYWCH2",
  "term_label": "Unknown biological process",
  "gene_name": "FLYWCH family member 2"
}